{
  "gene_symbol": "NOC4L",
  "term_id": "GO:0005730",
  "term_label": "nucleolus",
  "gene_name": "Nucleolar complex protein 4 homolog",
  "gene": "UniProtKB:Q9BVI4"
}